hypoglycin A gamma-glutamyl transpeptidase activity [GO:0102953] (molecular function) Definition: Catalysis of the reaction: glutathionate + hypoglycin A = L-cysteinylglycine + hypoglycin B. Sources: GOC:pz Relationships: is a type of aminoacyltransferase activity [GO:0016755]